acetylcholine catabolic process in synaptic cleft [GO:0001507] (biological process) Sources: GOC:ai Also known as: acetylcholine breakdown in synaptic cleft, acetylcholine degradation in synaptic cleft Relationships: is a type of acetylcholine catabolic process [GO:0006581]; is part of GO:0007271; occurs in synaptic cleft [GO:0043083] Definition: The chemical reactions and pathways resulting in the breakdown of acetylcholine that occurs in the synaptic cleft during synaptic transmission.